taurochenodeoxycholate 6alpha-hydroxylase activity [GO:0033780] (molecular function) Sources: EC:1.14.14.57 Also known as: CYP3A4, CYP4A21, taurochenodeoxycholate 6alpha-monooxygenase activity, taurochenodeoxycholate,NADPH:oxygen oxidoreductase (6alpha-hydroxylating) activity Definition: Catalysis of the reaction: taurochenodeoxycholate + O2 + reduced [NADPH--hemoprotein reductase] +  = taurohyocholate H+ + H2O + oxidized [NADPH--hemoprotein reductase]. Acts on taurochenodeoxycholate, taurodeoxycholate and less readily on lithocholate and chenodeoxycholate. Relationships: is a type of GO:0016712